{
  "term_id": "GO:0005634",
  "gene_symbol": "ZRANB1",
  "gene": "UniProtKB:Q9UGI0",
  "term_label": "nucleus",
  "gene_name": "Ubiquitin thioesterase ZRANB1"
}